UDP-beta-L-arabinofuranose import into Golgi lumen [GO:0140821] (biological process) Also known as: cytosol to Golgi apparatus UDP-beta-L-arabinofuranose transport Definition: The directed movement of UDP-beta-L-arabinofuranose from the cytosol to the Golgi apparatus of a cell. Relationships: is a type of organic anion transport [GO:0015711]; is a type of pyrimidine nucleotide-sugar transmembrane transport [GO:0090481]; is a type of GO:0140820 References: PMID:28373556